{
  "gene_name": "Ubiquitin-conjugating enzyme E2 U",
  "gene_symbol": "UBE2U",
  "gene": "UniProtKB:Q5VVX9",
  "term_label": "protein polyubiquitination",
  "term_id": "GO:0000209"
}